{
  "term_label": "Unknown biological process",
  "gene_name": "Plasminogen activator inhibitor 2",
  "gene_symbol": "SERPINB2",
  "gene": "UniProtKB:P05120",
  "term_id": "UNKNOWN:0002"
}